{
  "term_id": "UNKNOWN:0002",
  "term_label": "Unknown biological process",
  "gene": "UniProtKB:O43657",
  "gene_symbol": "TSPAN6",
  "gene_name": "Tetraspanin-6"
}